{
  "gene_name": "Receptor tyrosine-protein kinase erbB-3",
  "gene_symbol": "ERBB3",
  "gene": "UniProtKB:P21860",
  "term_id": "GO:0030182",
  "term_label": "neuron differentiation"
}